{
  "term_label": "NAD(P)H dehydrogenase (quinone) activity",
  "term_id": "GO:0003955",
  "gene_name": "NAD(P)H dehydrogenase [quinone] 1",
  "gene_symbol": "NQO1",
  "gene": "UniProtKB:P15559"
}